{
  "gene_symbol": "CCZ1B",
  "gene_name": "Vacuolar fusion protein CCZ1 homolog B",
  "gene": "UniProtKB:P86790",
  "term_label": "vesicle-mediated transport",
  "term_id": "GO:0016192"
}